{
  "gene": "UniProtKB:P54619",
  "term_id": "GO:0005737",
  "gene_name": "5'-AMP-activated protein kinase subunit gamma-1",
  "term_label": "cytoplasm",
  "gene_symbol": "PRKAG1"
}